cell leading edge [GO:0031252] (cellular component) Sources: GOC:pg Subtypes: growth cone leading edge [GO:0061850], leading edge of lamellipodium [GO:0061851] Relationships: is a type of GO:0110165 Also known as: front of cell, leading edge of cell Definition: The area of a motile cell closest to the direction of movement.